positive regulation of anion channel activity [GO:1901529] (biological process) Sources: GOC:TermGenie Definition: Any process that activates or increases the frequency, rate or extent of anion channel activity. Relationships: is a type of positive regulation of ion transmembrane transporter activity [GO:0032414]; is a type of GO:1903961; positively regulates GO:0005253 Also known as: up regulation of anion channel activity, up-regulation of anion channel activity, upregulation of anion channel activity, activation of anion channel activity Subtypes: positive regulation of voltage-gated chloride channel activity [GO:1902943]